{
  "gene": "UniProtKB:Q9NZD2",
  "term_label": "intermembrane lipid transfer",
  "gene_name": "Glycolipid transfer protein",
  "gene_symbol": "GLTP",
  "term_id": "GO:0120009"
}